{
  "term_id": "GO:0004305",
  "gene_symbol": "CHKA",
  "term_label": "ethanolamine kinase activity",
  "gene": "UniProtKB:P35790",
  "gene_name": "Choline kinase alpha"
}